{
  "term_label": "mRNA binding",
  "gene": "UniProtKB:P42766",
  "term_id": "GO:0003729",
  "gene_symbol": "RPL35",
  "gene_name": "Large ribosomal subunit protein uL29"
}